{
  "term_label": "regulation of transcription by RNA polymerase II",
  "gene_symbol": "ZNF599",
  "gene": "UniProtKB:Q96NL3",
  "term_id": "GO:0006357",
  "gene_name": "Zinc finger protein 599"
}